{
  "gene_symbol": "RHOU",
  "gene_name": "Rho-related GTP-binding protein RhoU",
  "term_id": "GO:0007015",
  "term_label": "actin filament organization",
  "gene": "UniProtKB:Q7L0Q8"
}